NAD+-protein mono-ADP-ribosyltransferase activity [GO:1990404] (MF) Subtypes: NAD+-protein-arginine ADP-ribosyltransferase activity [GO:0106274], NAD+-protein-C-terminal glycine ADP-ribosyltransferase activity [GO:0140802], NAD+-protein-cysteine ADP-ribosyltransferase activity [GO:0140803], NAD+-protein-lysine ADP-ribosyltransferase activity [GO:0140804], NAD+-protein-serine ADP-ribosyltransferase activity [GO:0140805], NAD+-protein-aspartate ADP-ribosyltransferase activity [GO:0140806], GO:0140807, NAD+-protein-tyrosine ADP-ribosyltransferase activity [GO:0140808], NAD+-protein-histidine ADP-ribosyltransferase activity [GO:0140815] References: PMID:1899243 Also known as: NAD+ ADP-ribosyltransferase activity, NAD+-protein ADP-ribosyltransferase activity, protein ADP-ribosyltransferase activity, ribosylase activity, protein ADP-ribosylase activity, protein mono-ADP-ribosyltransferase activity Regulation: regulated by regulation of protein ADP-ribosylation [GO:0010835]; negatively regulated by GO:0010836 Relationships: is_a pentosyltransferase activity [GO:0016763]; is a type of catalytic activity, acting on a protein [GO:0140096] Definition: Catalysis of the reaction: amino acyl-[protein] + NAD+ = H+ + (ADP-D-ribosyl)-amino acyl-[protein] + nicotinamide.